{
  "gene_symbol": "BMP6",
  "term_id": "GO:0005125",
  "term_label": "cytokine activity",
  "gene_name": "Bone morphogenetic protein 6",
  "gene": "UniProtKB:P22004"
}